{
  "gene_symbol": "HTR3E",
  "gene_name": "5-hydroxytryptamine receptor 3E",
  "gene": "UniProtKB:A5X5Y0",
  "term_label": "neuron projection",
  "term_id": "GO:0043005"
}